{
  "gene_symbol": "TAS1R2",
  "gene": "UniProtKB:Q8TE23",
  "gene_name": "Taste receptor type 1 member 2",
  "term_label": "sweet taste receptor activity",
  "term_id": "GO:0033041"
}